clathrin-sculpted vesicle [GO:0060198] (cellular component) Sources: GOC:dph Relationships: is a type of clathrin-coated vesicle [GO:0030136] Subtypes: clathrin-sculpted glutamate transport vesicle [GO:0060199], clathrin-sculpted acetylcholine transport vesicle [GO:0060200], clathrin-sculpted gamma-aminobutyric acid transport vesicle [GO:0061200], GO:0070081 Also known as: clathrin sculpted vesicle Definition: A clathrin-sculpted lipid bilayer membrane-enclosed vesicle after clathrin release.